{
  "gene": "UniProtKB:Q8N715",
  "term_label": "Unknown biological process",
  "gene_name": "Coiled-coil domain-containing protein 185",
  "term_id": "UNKNOWN:0002",
  "gene_symbol": "CCDC185"
}